synaptic vesicle membrane organization [GO:0048499] (biological process) Also known as: synaptic vesicle membrane organisation, SLMV biogenesis, synaptic vesicle membrane organization and biogenesis Subtypes: synaptic vesicle fusion to presynaptic active zone membrane [GO:0031629] Regulation: regulated by GO:1901632; negatively regulated by negative regulation of synaptic vesicle membrane organization [GO:1901633]; positively regulated by GO:1901634 References: PMID:10620806 Sources: GOC:dph, GOC:jl, GOC:mah Definition: A process that is carried out at the cellular level which results in the assembly, arrangement of constituent parts, or disassembly of the membrane surrounding a synaptic vesicle. Relationships: is a type of membrane organization [GO:0061024]; is part of GO:0010256